disproportionation of elemental sulfur [GO:0019422] (biological process) Relationships: is_a sulfur compound metabolic process [GO:0006790] Also known as: disproportionation of elemental sulphur Sources: MetaCyc:P203-PWY Definition: The process in which sulfur compounds with an intermediate oxidation state serve as both electron donors and electron acceptors in an energy-generating redox process. The reaction takes place anaerobically, in light and in the absence of CO2.